pulmonary valve development [GO:0003177] (biological process) Sources: GOC:mtg_heart Definition: The progression of the pulmonary valve over time, from its formation to the mature structure. Relationships: is a type of semi-lunar valve development [GO:1905314]